{
  "gene": "UniProtKB:Q9GZP0",
  "gene_symbol": "PDGFD",
  "term_label": "positive regulation of ERK1 and ERK2 cascade",
  "term_id": "GO:0070374",
  "gene_name": "Platelet-derived growth factor D"
}